negative regulation of chemokine (C-C motif) ligand 20 production [GO:1903885] (biological process) Definition: Any process that stops, prevents or reduces the frequency, rate or extent of chemokine (C-C motif) ligand 20 production. Also known as: down regulation of C-C motif chemokine 20 production, down regulation of CCL-20 production, down regulation of CCL20 production, down regulation of chemokine (C-C motif) ligand 20 production, down-regulation of C-C motif chemokine 20 production, down-regulation of CCL-20 production, down-regulation of CCL20 production, down-regulation of chemokine (C-C motif) ligand 20 production, downregulation of C-C motif chemokine 20 production, downregulation of CCL-20 production, downregulation of CCL20 production, downregulation of chemokine (C-C motif) ligand 20 production, negative regulation of C-C motif chemokine 20 production, negative regulation of CCL-20 production, negative regulation of CCL20 production, inhibition of C-C motif chemokine 20 production, inhibition of CCL-20 production, inhibition of CCL20 production, inhibition of chemokine (C-C motif) ligand 20 production References: PMID:20054338 Sources: GOC:TermGenie, GOC:krc, GO_REF:0000058 Relationships: is a type of negative regulation of chemokine production [GO:0032682]; is a type of GO:1903884; negatively regulates chemokine (C-C motif) ligand 20 production [GO:0036392]